manganese:proton antiporter activity [GO:0010486] (molecular function) Definition: Enables the transfer of a solute or solutes from one side of a membrane to the other according to the reaction: Mn2+(in) + H+(out) = Mn2+(out) + H+(in). Also known as: manganese:hydrogen antiporter activity References: PMID:17559518 Relationships: is a type of GO:0005384; is a type of metal cation:proton antiporter activity [GO:0051139]